{
  "gene": "UniProtKB:Q9Y2K2",
  "gene_symbol": "SIK3",
  "term_label": "cytoplasm",
  "term_id": "GO:0005737",
  "gene_name": "Serine_threonine-protein kinase SIK3"
}